{
  "term_label": "lipoprotein transport",
  "gene_name": "Protein unc-119 homolog A",
  "term_id": "GO:0042953",
  "gene": "UniProtKB:Q13432",
  "gene_symbol": "UNC119"
}